{
  "gene_symbol": "TKTL2",
  "gene_name": "Transketolase-like protein 2",
  "term_id": "GO:0004802",
  "term_label": "transketolase activity",
  "gene": "UniProtKB:Q9H0I9"
}